{
  "gene_name": "V-type proton ATPase subunit d 2",
  "term_id": "GO:0016471",
  "gene": "UniProtKB:Q8N8Y2",
  "gene_symbol": "ATP6V0D2",
  "term_label": "vacuolar proton-transporting V-type ATPase complex"
}